{
  "gene_symbol": "GAGE12E",
  "term_label": "Unknown biological process",
  "gene_name": "G antigen 12B_C_D_E",
  "gene": "UniProtKB:A1L429",
  "term_id": "UNKNOWN:0002"
}